lipo-chitin oligosaccharide transmembrane transporter activity [GO:1901513] (molecular function) Sources: GOC:TermGenie Relationships: is a type of transmembrane transporter activity [GO:0022857] Definition: Enables the transfer of lipo-chitin oligosaccharide from one side of a membrane to the other. Subtypes: ATPase-coupled lipo-chitin oligosaccharide transmembrane transporter activity [GO:1901514]